{
  "term_id": "GO:0045202",
  "gene_symbol": "C1QL3",
  "term_label": "synapse",
  "gene": "UniProtKB:Q5VWW1",
  "gene_name": "Complement C1q-like protein 3"
}